{
  "gene": "UniProtKB:P00533",
  "term_label": "basal plasma membrane",
  "gene_symbol": "EGFR",
  "gene_name": "Epidermal growth factor receptor",
  "term_id": "GO:0009925"
}